{
  "term_id": "GO:0072686",
  "gene_name": "CLIP-associating protein 1",
  "gene": "UniProtKB:Q7Z460",
  "term_label": "mitotic spindle",
  "gene_symbol": "CLASP1"
}